{
  "term_label": "glutathione transferase activity",
  "term_id": "GO:0004364",
  "gene": "UniProtKB:P09488",
  "gene_symbol": "GSTM1",
  "gene_name": "Glutathione S-transferase Mu 1"
}